1-phosphatidylinositol-4-phosphate 5-kinase activity [GO:0016308] (molecular function) Sources: EC:2.7.1.68, RHEA:14425 Relationships: is a type of GO:0052742 Also known as: 1-phosphatidylinositol-4-phosphate kinase activity, PIP kinase activity, diphosphoinositide kinase activity, phosphatidylinositol 4-phosphate kinase activity, PIP5K, 1-phosphatidylinositol-4-phosphate kinase, class IA, 1-phosphatidylinositol-4-phosphate kinase, class IB, type I PIP kinase activity, ATP:1-phosphatidyl-1D-myo-inositol-4-phosphate 5-phosphotransferase activity, PI(4)5K, PtdIns(4)P-5-kinase activity, phosphatidylinositol-4-phosphate 5-kinase activity Definition: Catalysis of the reaction: a 1-phosphatidyl-1D-myo-inositol 4-phosphate + ATP = a 1-phosphatidyl-1D-myo-inositol 4,5-bisphosphate + ADP + H+.